negative regulation of intracellular protein transport [GO:0090317] (BP) Sources: GOC:tb Relationships: is a type of GO:0032387; is a type of GO:0033157; is a type of GO:0051224; negatively regulates intracellular protein transport [GO:0006886] Subtypes: GO:0042308, negative regulation of protein export from nucleus [GO:0046826], negative regulation of protein exit from endoplasmic reticulum [GO:0070862], negative regulation of post-translational protein targeting to membrane, translocation [GO:0120236], GO:1900484, negative regulation of protein targeting to vacuole involved in autophagy [GO:1904052], negative regulation of axo-dendritic protein transport [GO:1905127], negative regulation of endosome to plasma membrane protein transport [GO:1905750] Definition: Any process that decreases the frequency, rate or extent of the directed movement of proteins within cells.